{
  "term_id": "GO:0060271",
  "term_label": "cilium assembly",
  "gene_name": "IQ and ubiquitin-like domain-containing protein",
  "gene": "UniProtKB:Q8NA54",
  "gene_symbol": "IQUB"
}